{
  "gene_name": "Ankyrin repeat and BTB_POZ domain-containing protein 1",
  "term_id": "GO:0000151",
  "gene_symbol": "ABTB1",
  "gene": "UniProtKB:Q969K4",
  "term_label": "ubiquitin ligase complex"
}